{
  "gene_symbol": "MIS18BP1",
  "term_label": "chromosome, centromeric region",
  "gene": "UniProtKB:Q6P0N0",
  "term_id": "GO:0000775",
  "gene_name": "Mis18-binding protein 1"
}